{
  "gene_symbol": "ANP32D",
  "term_id": "UNKNOWN:0002",
  "term_label": "Unknown biological process",
  "gene_name": "Acidic leucine-rich nuclear phosphoprotein 32 family member D",
  "gene": "UniProtKB:O95626"
}